BRCA1-Rad51 complex [GO:0070767] (cellular component) Definition: A protein complex that contains BRCA1 and Rad 51, and is involved in the control of recombination and of genome integrity. Relationships: is a type of nuclear protein-containing complex [GO:0140513] References: PMID:9008167 Sources: GOC:mah